{
  "term_label": "chemorepellent activity",
  "gene_symbol": "SEMA6C",
  "term_id": "GO:0045499",
  "gene": "UniProtKB:Q9H3T2",
  "gene_name": "Semaphorin-6C"
}